{
  "gene": "UniProtKB:P55064",
  "gene_symbol": "AQP5",
  "term_label": "apical plasma membrane",
  "term_id": "GO:0016324",
  "gene_name": "Aquaporin-5"
}